{
  "term_label": "endoplasmic reticulum membrane",
  "gene_name": "Reticulon-4",
  "term_id": "GO:0005789",
  "gene_symbol": "RTN4",
  "gene": "UniProtKB:Q9NQC3"
}